{
  "gene_name": "GRB2-associated and regulator of MAPK protein 2",
  "term_id": "UNKNOWN:0003",
  "term_label": "Unknown cellular component",
  "gene_symbol": "GAREM2",
  "gene": "UniProtKB:Q75VX8"
}